{
  "term_id": "GO:0019216",
  "gene": "UniProtKB:Q9H6K4",
  "gene_name": "Optic atrophy 3 protein",
  "gene_symbol": "OPA3",
  "term_label": "regulation of lipid metabolic process"
}